{
  "term_label": "protein kinase activity",
  "gene": "UniProtKB:Q9H792",
  "gene_name": "Inactive tyrosine-protein kinase PEAK1",
  "term_id": "GO:0004672",
  "gene_symbol": "PEAK1"
}